chloroplast membrane [GO:0031969] (cellular component) Definition: Either of the lipid bilayers that surround a chloroplast and form the chloroplast envelope. Sources: GOC:mah, GOC:pz Relationships: is a type of plastid membrane [GO:0042170]; is part of GO:0009941 Subtypes: chloroplast inner membrane [GO:0009706], chloroplast outer membrane [GO:0009707]